{
  "term_label": "mitotic cell cycle",
  "term_id": "GO:0000278",
  "gene": "UniProtKB:Q9H4B7",
  "gene_name": "Tubulin beta-1 chain",
  "gene_symbol": "TUBB1"
}